symbiont-mediated perturbation of host cytoskeleton [GO:0052039] (biological process) Sources: GOC:mtg_pamgo_17jul06 Definition: The process in which an organism effects a change that impairs the structure or function of the host cytoskeleton. The host is defined as the larger of the organisms involved in a symbiotic interaction. Also known as: perturbation by symbiont of host cytoskeleton, rounding by symbiont of host cells, disruption by symbiont of host cytoskeleton, modification by symbiont of host cytoskeleton Relationships: is a type of GO:0052008 Subtypes: symbiont-mediated perturbation of host actin cytoskeleton [GO:0141027], GO:0141028